{
  "term_id": "GO:0008188",
  "gene_name": "Gastrin-releasing peptide receptor",
  "gene_symbol": "GRPR",
  "term_label": "neuropeptide receptor activity",
  "gene": "UniProtKB:P30550"
}